regulation of vitamin E biosynthetic process [GO:1904965] (biological process) Definition: Any process that modulates the frequency, rate or extent of vitamin E biosynthetic process. References: PMID:20823244 Sources: GOC:TermGenie, GO_REF:0000058 Also known as: regulation of tocopherol biosynthesis, regulation of tocopherol biosynthetic process, regulation of vitamin E anabolism, regulation of vitamin E biosynthesis, regulation of vitamin E formation, regulation of vitamin E synthesis, regulation of alpha-tocopherol biosynthesis, regulation of alpha-tocopherol biosynthetic process Relationships: is a type of regulation of biosynthetic process [GO:0009889]; is a type of GO:0030656; regulates vitamin E biosynthetic process [GO:0010189] Subtypes: positive regulation of vitamin E biosynthetic process [GO:1904966]